{
  "gene_name": "Proprotein convertase subtilisin_kexin type 7",
  "term_label": "trans-Golgi network",
  "term_id": "GO:0005802",
  "gene": "UniProtKB:Q16549",
  "gene_symbol": "PCSK7"
}